{
  "term_label": "aryl hydrocarbon receptor complex",
  "gene_name": "Aryl hydrocarbon receptor nuclear translocator",
  "gene": "UniProtKB:P27540",
  "gene_symbol": "ARNT",
  "term_id": "GO:0034751"
}